{
  "gene": "UniProtKB:P57073",
  "gene_name": "Transcription factor SOX-8",
  "term_label": "morphogenesis of an epithelium",
  "gene_symbol": "SOX8",
  "term_id": "GO:0002009"
}